{
  "gene_name": "NAD-dependent protein deacylase sirtuin-5, mitochondrial",
  "term_id": "GO:0061697",
  "gene_symbol": "SIRT5",
  "term_label": "protein-glutaryllysine deglutarylase activity",
  "gene": "UniProtKB:Q9NXA8"
}